isocitrate O-dihydroxycinnamoyltransferase activity [GO:0047168] (molecular function) Sources: EC:2.3.1.126, RHEA:20756 Definition: Catalysis of the reaction: caffeoyl-CoA + isocitrate = 2-caffeoylisocitrate + CoA. Also known as: caffeoyl-CoA:isocitrate 3-O-(3,4-dihydroxycinnamoyl)transferase activity Relationships: is a type of acyltransferase activity, transferring groups other than amino-acyl groups [GO:0016747]